{
  "gene_symbol": "CISH",
  "term_label": "cytokine receptor binding",
  "gene": "UniProtKB:Q9NSE2",
  "term_id": "GO:0005126",
  "gene_name": "Cytokine-inducible SH2-containing protein"
}